{
  "gene_symbol": "SPATA4",
  "term_id": "GO:0051493",
  "term_label": "regulation of cytoskeleton organization",
  "gene": "UniProtKB:Q8NEY3",
  "gene_name": "Spermatogenesis-associated protein 4"
}